{
  "gene_symbol": "SLC35G3",
  "gene": "UniProtKB:Q8N808",
  "term_id": "UNKNOWN:0001",
  "gene_name": "Solute carrier family 35 member G3",
  "term_label": "Unknown molecular function"
}